{
  "term_label": "plasma membrane",
  "gene": "UniProtKB:Q86UE6",
  "term_id": "GO:0005886",
  "gene_symbol": "LRRTM1",
  "gene_name": "Leucine-rich repeat transmembrane neuronal protein 1"
}